{
  "gene_name": "Growth factor receptor-bound protein 2",
  "term_label": "phosphotyrosine residue binding",
  "gene_symbol": "GRB2",
  "term_id": "GO:0001784",
  "gene": "UniProtKB:P62993"
}